{
  "gene": "UniProtKB:Q16589",
  "gene_symbol": "CCNG2",
  "term_label": "cytoplasm",
  "term_id": "GO:0005737",
  "gene_name": "Cyclin-G2"
}